transport [GO:0006810] (biological process) Note: Note that this term should not be used for direct annotation. It should be possible to make a more specific annotation to one of the children of this term, for e.g. to transmembrane transport, to microtubule-based transport or to vesicle-mediated transport. Relationships: is a type of establishment of localization [GO:0051234] Definition: The directed movement of substances (such as macromolecules, small molecules, ions) or cellular components (such as complexes and organelles) into, out of or within a cell, or between cells, or within a multicellular organism by means of some agent such as a transporter or a transporter complex, a pore or a motor protein. Sources: GOC:dos, GOC:dph, GOC:jl, GOC:mah Also known as: single-organism transport Subtypes: monoatomic ion transport [GO:0006811], GO:0006836, eye pigment precursor transport [GO:0006856], extracellular transport [GO:0006858], amino acid transport [GO:0006865], lipid transport [GO:0006869], GO:0007300, carbohydrate transport [GO:0008643], GO:0009914, vascular transport [GO:0010232], intercellular transport [GO:0010496], gas transport [GO:0015669], organic cation transport [GO:0015695], inorganic anion transport [GO:0015698], arsenite transport [GO:0015700], GO:0015711, mevalonate transport [GO:0015728], GO:0015748, organic acid transport [GO:0015849], organic hydroxy compound transport [GO:0015850], alkane transport [GO:0015895], vesicle-mediated transport [GO:0016192], one-carbon compound transport [GO:0019755], vesicle cargo loading [GO:0035459], synaptic vesicle recycling [GO:0036465], fluid transport [GO:0042044], xenobiotic transport [GO:0042908], GO:0046903, intracellular transport [GO:0046907], GO:0048489, vitamin transport [GO:0051180], GO:0051625, GO:0051904, GO:0055085, transepithelial transport [GO:0070633], nitrogen compound transport [GO:0071705], sulfur compound transport [GO:0072348], cutin transport [GO:0080051], import into cell [GO:0098657], GO:0099111, export from cell [GO:0140352], paracellular transport [GO:0160184], carbohydrate derivative transport [GO:1901264], GO:1901374, flavonoid transport from endoplasmic reticulum to plant-type vacuole [GO:1903415] Regulation: regulated by regulation of transport [GO:0051049]; positively regulated by positive regulation of transport [GO:0051050]; negatively regulated by negative regulation of transport [GO:0051051]